{
  "gene_symbol": "TUBB8",
  "term_id": "GO:0000278",
  "gene": "UniProtKB:Q3ZCM7",
  "gene_name": "Tubulin beta-8 chain",
  "term_label": "mitotic cell cycle"
}